{
  "gene": "UniProtKB:B1AK76",
  "term_id": "UNKNOWN:0001",
  "gene_name": "Putative SNURF-like protein",
  "term_label": "Unknown molecular function",
  "gene_symbol": "SNURFL"
}